{
  "gene_symbol": "CYP4F3",
  "term_label": "phylloquinone catabolic process",
  "term_id": "GO:0042376",
  "gene": "UniProtKB:Q08477",
  "gene_name": "Cytochrome P450 4F3"
}